{
  "gene_symbol": "ASB8",
  "gene_name": "Ankyrin repeat and SOCS box protein 8",
  "gene": "UniProtKB:Q9H765",
  "term_id": "UNKNOWN:0003",
  "term_label": "Unknown cellular component"
}